succinate dehydrogenase (quinone) activity [GO:0008177] (molecular function) Definition: Catalysis of the reaction: a quinone + succinate = a quinol + fumarate. Relationships: is_a succinate dehydrogenase activity [GO:0000104]; is a type of oxidoreductase activity, acting on the CH-CH group of donors, quinone or related compound as acceptor [GO:0016635] Also known as: succinic dehydrogenase activity, fumarate reductase (menaquinone), succinate dehydrogenase (menaquinone), succinate dehydrogenase (ubiquinone) activity Sources: RHEA:40523